pancreatic D cell fate commitment [GO:0003328] (biological process) Definition: The commitment of a cell to a pancreatic D cell fate and its capacity to differentiate into a pancreatic D cell. A delta cell is a cell of the pancreas that produces somatostatin. Relationships: is a type of neuron fate commitment [GO:0048663]; is a type of GO:0072148; is part of pancreatic D cell differentiation [GO:0003311] Sources: GOC:dph